{
  "term_id": "GO:0005923",
  "term_label": "bicellular tight junction",
  "gene_symbol": "MARVELD2",
  "gene": "UniProtKB:Q8N4S9",
  "gene_name": "MARVEL domain-containing protein 2"
}